{
  "gene_name": "Cytosolic 5'-nucleotidase 1B",
  "term_label": "adenosine metabolic process",
  "gene": "UniProtKB:Q96P26",
  "gene_symbol": "NT5C1B",
  "term_id": "GO:0046085"
}